{
  "term_id": "GO:0007155",
  "term_label": "cell adhesion",
  "gene_name": "Protocadherin alpha-13",
  "gene": "UniProtKB:Q9Y5I0",
  "gene_symbol": "PCDHA13"
}